{
  "term_id": "GO:0000151",
  "term_label": "ubiquitin ligase complex",
  "gene_symbol": "UBE3D",
  "gene_name": "E3 ubiquitin-protein ligase E3D",
  "gene": "UniProtKB:Q7Z6J8"
}